{
  "term_label": "cell differentiation",
  "gene": "UniProtKB:P13056",
  "gene_symbol": "NR2C1",
  "term_id": "GO:0030154",
  "gene_name": "Nuclear receptor subfamily 2 group C member 1"
}